{
  "gene_symbol": "POTEF",
  "gene": "UniProtKB:A5A3E0",
  "term_label": "axonogenesis",
  "term_id": "GO:0007409",
  "gene_name": "POTE ankyrin domain family member F"
}